electron transport coupled proton transport [GO:0015990] (BP) Relationships: is a type of energy coupled proton transmembrane transport, against electrochemical gradient [GO:0015988] Definition: The transport of protons against an electrochemical gradient, using energy from electron transport. Sources: GOC:mah